{
  "gene_symbol": "FAM171B",
  "gene": "UniProtKB:Q6P995",
  "term_id": "UNKNOWN:0001",
  "gene_name": "Protein FAM171B",
  "term_label": "Unknown molecular function"
}